{
  "gene": "UniProtKB:Q96G30",
  "term_label": "regulation of adenylate cyclase-activating G protein-coupled receptor signaling pathway",
  "gene_symbol": "MRAP2",
  "gene_name": "Melanocortin-2 receptor accessory protein 2",
  "term_id": "GO:0106070"
}